regulation of protein localization to cell-cell junction [GO:0150106] (biological process) Definition: Any process that modulates the frequency, rate or extent of protein localization to cell-cell junction. References: PMID:26706435 Sources: GOC:aruk, GOC:bc Relationships: is a type of regulation of protein localization [GO:0032880]; regulates protein localization to cell-cell junction [GO:0150105] Subtypes: GO:0150107, negative regulation of protein localization to cell-cell junction [GO:0150119], regulation of protein localization to adherens junction [GO:1904702]